plant parenchymal cell differentiation [GO:0048760] (biological process) Definition: The process in which a relatively unspecialized cell acquires specialized features of a parenchymal cell. Parenchymal cells are the most abundant and versatile cells in plants. They have very few distinguishing characteristics and botanists classify them as any cell type that cannot be assigned to any other structural or functional class. They can redifferentiate and dedifferentiate and are involved in storage, basic metabolism and other processes. The cells are polyhedral, typically with thin, non-lignified cellulose cell walls and nucleate living protoplasm. They vary in size, form, and wall structure. Sources: CL:0000668, GOC:jid, ISBN:069716957X, PO:0005421 Also known as: parenchymal cell differentiation Relationships: is a type of cell differentiation [GO:0030154] Subtypes: companion cell differentiation [GO:0048758]